{
  "gene": "UniProtKB:Q96PZ0",
  "term_id": "GO:0005634",
  "term_label": "nucleus",
  "gene_name": "Pseudouridylate synthase 7 homolog",
  "gene_symbol": "PUS7"
}